{
  "term_id": "GO:0005254",
  "term_label": "chloride channel activity",
  "gene_symbol": "GABRA4",
  "gene": "UniProtKB:P48169",
  "gene_name": "Gamma-aminobutyric acid receptor subunit alpha-4"
}